central tolerance induction to self antigen [GO:0002509] (BP) Relationships: is a type of GO:0002508; is a type of tolerance induction to self antigen [GO:0002513] Definition: Tolerance induction in the central lymphoid organs directed at self antigens. References: PMID:16460922 Sources: GOC:jal, ISBN:0781735149